{
  "gene_name": "Selenocysteine insertion sequence-binding protein 2",
  "gene": "UniProtKB:Q96T21",
  "term_id": "GO:0001514",
  "gene_symbol": "SECISBP2",
  "term_label": "selenocysteine incorporation"
}